{
  "gene_name": "Estrogen receptor",
  "term_label": "nuclear receptor activity",
  "term_id": "GO:0004879",
  "gene_symbol": "ESR1",
  "gene": "UniProtKB:P03372"
}